{
  "term_label": "Unknown biological process",
  "gene_name": "MORF4 family-associated protein 1-like 1",
  "term_id": "UNKNOWN:0002",
  "gene_symbol": "MRFAP1L1",
  "gene": "UniProtKB:Q96HT8"
}